DNA recombinase assembly [GO:0000730] (biological process) Relationships: is a type of protein-DNA complex assembly [GO:0065004]; is a type of GO:0090735; is part of GO:0045003 References: PMID:10357855 Definition: The aggregation, arrangement and bonding together of strand exchange proteins (recombinases) into higher order oligomers on single-stranded DNA. Also known as: Rad51 nucleoprotein filament formation Subtypes: meiotic DNA recombinase assembly [GO:0000707]